{
  "gene": "UniProtKB:A0A2R8YD15",
  "gene_symbol": "A0A2R8YD15",
  "gene_name": "Uncharacterized protein",
  "term_label": "Unknown molecular function",
  "term_id": "UNKNOWN:0001"
}